{
  "term_id": "GO:0019901",
  "gene": "UniProtKB:P63000",
  "gene_symbol": "RAC1",
  "gene_name": "Ras-related C3 botulinum toxin substrate 1",
  "term_label": "protein kinase binding"
}